molecular tag activity [GO:0141047] (MF) Relationships: is a type of molecular_function [GO:0003674] Also known as: covalent modifier, tag Note: Use this term to annotate conjugated tags, not for conjugating enzymes. At the time of writing, all known gene products with this activity are ubiquitin-like, either based on overall sequence similarity or the presence of common motifs and structures. Definition: A molecular function exhibited by a protein that is covalently attached (AKA tagged or conjugated) to another molecule (for example a protein or a lipid) where it acts as a marker, recognized by the cellular apparatus to target the tagged protein for some cellular process such as modification, sequestration, transport or degradation. Subtypes: protein tag activity [GO:0031386], membrane tag activity [GO:0141048] References: PMID:17632063